{
  "gene_name": "R-spondin-4",
  "gene_symbol": "RSPO4",
  "term_label": "extracellular space",
  "term_id": "GO:0005615",
  "gene": "UniProtKB:Q2I0M5"
}